negative regulation of auxin mediated signaling pathway [GO:0010930] (biological process) Definition: Any process that decreases the rate, frequency or extent of auxin mediated signaling pathway. Auxin mediated signaling pathway is the series of molecular signals generated in response to detection of auxin. Relationships: is a type of negative regulation of signal transduction [GO:0009968]; is a type of regulation of auxin mediated signaling pathway [GO:0010928]; negatively regulates auxin-activated signaling pathway [GO:0009734] Also known as: negative regulation of auxin mediated signalling pathway Sources: GOC:dph, GOC:tb